{
  "gene": "UniProtKB:P29275",
  "term_label": "adenylate cyclase-activating G protein-coupled receptor signaling pathway",
  "gene_name": "Adenosine receptor A2b",
  "term_id": "GO:0007189",
  "gene_symbol": "ADORA2B"
}